(S)-limonene 3-monooxygenase activity [GO:0018674] (molecular function) Sources: RHEA:15129 Definition: Catalysis of the reaction: (4S)-limonene + O2 + reduced [NADPH--hemoprotein reductase] = (1S,6R)-isopiperitenol + H+ + H2O + oxidized [NADPH--hemoprotein reductase]. Relationships: is a type of oxidoreductase activity, acting on paired donors, with incorporation or reduction of molecular oxygen, reduced flavin or flavoprotein as one donor, and incorporation of one atom of oxygen [GO:0016712]; is a type of limonene monooxygenase activity [GO:0019113] Also known as: (-)-limonene 3-monooxygenase activity, limonene 3-hydroxylase activity, (-)-limonene 3-hydroxylase activity, (-)-limonene,NADPH:oxygen oxidoreductase (3-hydroxylating) activity, (S)-limonene,NADPH:oxygen oxidoreductase (3-hydroxylating)